{
  "gene": "UniProtKB:O15079",
  "term_id": "GO:0005881",
  "gene_symbol": "SNPH",
  "term_label": "cytoplasmic microtubule",
  "gene_name": "Syntaphilin"
}